podosome core [GO:0061825] (cellular component) References: PMID:23158496 Definition: The F-actin-rich core of an adhesion structure characterized by formation upon cell substrate contact and localization at the substrate-attached part of the cell. Relationships: is a type of cellular anatomical structure [GO:0110165]; is part of podosome [GO:0002102]